{
  "gene_symbol": "POLR2F",
  "term_label": "transcription by RNA polymerase I",
  "term_id": "GO:0006360",
  "gene": "UniProtKB:P61218",
  "gene_name": "DNA-directed RNA polymerases I, II, and III subunit RPABC2"
}